{
  "gene": "UniProtKB:Q6UWP8",
  "term_label": "Unknown molecular function",
  "gene_name": "Suprabasin",
  "term_id": "UNKNOWN:0001",
  "gene_symbol": "SBSN"
}